{
  "gene_name": "A disintegrin and metalloproteinase with thrombospondin motifs 10",
  "gene_symbol": "ADAMTS10",
  "gene": "UniProtKB:Q9H324",
  "term_id": "GO:0030198",
  "term_label": "extracellular matrix organization"
}